{
  "term_id": "GO:0015031",
  "term_label": "protein transport",
  "gene_name": "Charged multivesicular body protein 2b",
  "gene_symbol": "CHMP2B",
  "gene": "UniProtKB:Q9UQN3"
}